{
  "gene": "UniProtKB:Q16627",
  "term_label": "chemokine activity",
  "term_id": "GO:0008009",
  "gene_name": "C-C motif chemokine 14",
  "gene_symbol": "CCL14"
}